{
  "gene_symbol": "SEPTIN14",
  "gene_name": "Septin-14",
  "gene": "UniProtKB:Q6ZU15",
  "term_label": "microtubule cytoskeleton",
  "term_id": "GO:0015630"
}